nucleocytoplasmic carrier activity [GO:0140142] (molecular function) Also known as: nucleocytoplasmic importin/exportin activity, miRNA transporter activity, pre-miRNA transporter activity Sources: GOC:pg Definition: Binding to and carrying a cargo between the nucleus and the cytoplasm by moving along with the cargo. The cargo can be either a RNA or a protein. Subtypes: nuclear export signal receptor activity [GO:0005049], nuclear import signal receptor activity [GO:0061608] Relationships: is a type of GO:0140104; is part of nucleocytoplasmic transport [GO:0006913]